{
  "gene": "UniProtKB:O60258",
  "term_id": "GO:0005105",
  "gene_symbol": "FGF17",
  "gene_name": "Fibroblast growth factor 17",
  "term_label": "type 1 fibroblast growth factor receptor binding"
}